negative regulation of cellular defense response [GO:0051245] (biological process) Definition: Any process that stops, prevents, or reduces the rate of the cellular defense response. Sources: GOC:ai Also known as: down regulation of cellular defense response, down-regulation of cellular defense response, downregulation of cellular defense response, negative regulation of cellular defence response, inhibition of cellular defense response Relationships: is a type of regulation of cellular defense response [GO:0010185]; is a type of negative regulation of defense response [GO:0031348]; negatively regulates cellular defense response [GO:0006968]